{
  "gene_name": "Nucleoredoxin-like protein 2",
  "gene": "UniProtKB:Q5VZ03",
  "gene_symbol": "NXNL2",
  "term_id": "UNKNOWN:0003",
  "term_label": "Unknown cellular component"
}